{
  "term_label": "spindle",
  "gene_symbol": "KIF2B",
  "term_id": "GO:0005819",
  "gene": "UniProtKB:Q8N4N8",
  "gene_name": "Kinesin-like protein KIF2B"
}